{
  "term_label": "fatty acid catabolic process",
  "gene": "UniProtKB:O00519",
  "gene_symbol": "FAAH",
  "term_id": "GO:0009062",
  "gene_name": "Fatty-acid amide hydrolase 1"
}